{
  "gene": "UniProtKB:O00341",
  "term_id": "GO:0005313",
  "gene_symbol": "SLC1A7",
  "term_label": "L-glutamate transmembrane transporter activity",
  "gene_name": "Excitatory amino acid transporter 5"
}